regulation of response to calcium ion [GO:1905945] (biological process) Also known as: regulation of response to Ca2+ ion Relationships: is a type of regulation of response to stimulus [GO:0048583]; regulates response to calcium ion [GO:0051592] Definition: Any process that modulates the frequency, rate or extent of response to calcium ion. References: PMID:11404397 Sources: GOC:TermGenie, GOC:aruk, GOC:bc, GO_REF:0000058 Subtypes: negative regulation of response to calcium ion [GO:1905946], GO:1905947